{
  "term_label": "cytoplasm",
  "term_id": "GO:0005737",
  "gene_name": "eIF5-mimic protein 1",
  "gene": "UniProtKB:Q9Y6E2",
  "gene_symbol": "BZW2"
}